developmental vegetative growth [GO:0080186] (biological process) Regulation: regulated by regulation of developmental vegetative growth [GO:1905613]; negatively regulated by negative regulation of developmental vegetative growth [GO:1905614]; positively regulated by GO:1905615 Subtypes: GO:0010448 Definition: The increase in size or mass of non-reproductive plant parts. Relationships: is a type of developmental growth [GO:0048589] Sources: PO:0007134